regulation of NLRP3 inflammasome complex assembly [GO:1900225] (biological process) Also known as: regulation of NALP3 inflammasome complex assembly, regulation of NLRP3 inflammasome activation Subtypes: negative regulation of NLRP3 inflammasome complex assembly [GO:1900226], positive regulation of NLRP3 inflammasome complex assembly [GO:1900227] Relationships: is a type of regulation of protein-containing complex assembly [GO:0043254]; is part of regulation of inflammasome-mediated signaling pathway [GO:0141085]; regulates GO:0044546 Definition: Any process that modulates the frequency, rate or extent of NLRP3 inflammasome complex assembly. Sources: GOC:TermGenie